{
  "gene": "UniProtKB:Q01362",
  "term_id": "GO:0009897",
  "term_label": "external side of plasma membrane",
  "gene_name": "High affinity immunoglobulin epsilon receptor subunit beta",
  "gene_symbol": "MS4A2"
}